{
  "term_label": "extracellular space",
  "gene": "UniProtKB:Q9H2R5",
  "gene_name": "Kallikrein-15",
  "gene_symbol": "KLK15",
  "term_id": "GO:0005615"
}